{
  "term_id": "UNKNOWN:0002",
  "gene_symbol": "CNIH1",
  "term_label": "Unknown biological process",
  "gene": "UniProtKB:O95406",
  "gene_name": "Protein cornichon homolog 1"
}